{
  "term_label": "nucleus",
  "gene": "UniProtKB:P26358",
  "term_id": "GO:0005634",
  "gene_symbol": "DNMT1",
  "gene_name": "DNA (cytosine-5)-methyltransferase 1"
}